{
  "term_id": "UNKNOWN:0002",
  "gene_symbol": "TANK",
  "gene_name": "TRAF family member-associated NF-kappa-B activator",
  "term_label": "Unknown biological process",
  "gene": "UniProtKB:Q92844"
}